{
  "gene_name": "Claudin-12",
  "gene": "UniProtKB:P56749",
  "term_label": "Unknown molecular function",
  "gene_symbol": "CLDN12",
  "term_id": "UNKNOWN:0001"
}